{
  "gene_symbol": "YPEL2",
  "gene_name": "Protein yippee-like 2",
  "term_label": "Unknown cellular component",
  "term_id": "UNKNOWN:0003",
  "gene": "UniProtKB:Q96QA6"
}